positive regulation of miRNA catabolic process [GO:2000627] (biological process) Definition: Any process that activates or increases the frequency, rate or extent of miRNA catabolic process. Sources: GOC:dph Also known as: positive regulation of microRNA catabolic process Relationships: is a type of positive regulation of catabolic process [GO:0009896]; is a type of regulation of miRNA catabolic process [GO:2000625]; is a type of positive regulation of miRNA metabolic process [GO:2000630]; positively regulates miRNA catabolic process [GO:0010587]